{
  "term_label": "axon development",
  "term_id": "GO:0061564",
  "gene_name": "Class E basic helix-loop-helix protein 23",
  "gene_symbol": "BHLHE23",
  "gene": "UniProtKB:Q8NDY6"
}